{
  "gene": "UniProtKB:Q8NGH7",
  "gene_symbol": "OR52L1",
  "gene_name": "Olfactory receptor 52L1",
  "term_id": "GO:0004984",
  "term_label": "olfactory receptor activity"
}